trypanothione biosynthetic process [GO:0019342] (biological process) Regulation: regulated by regulation of trypanothione biosynthetic process [GO:1905722]; negatively regulated by negative regulation of trypanothione biosynthetic process [GO:1905723]; RO_0002213 by positive regulation of trypanothione biosynthetic process [GO:1905724] Definition: The chemical reactions and pathways resulting in the formation of trypanothione (N1,N6,-bis(glutathionyl)spermidine) in two steps from glutathione and spermidine via an N1- or N8-glutathionylspermidine intermediate. Trypanothione appears to be an essential redox intermediate in intracellular thiol redox regulation. It also plays a role in protecting against oxidative stress. References: PMID:9677355 Sources: MetaCyc:TRYPANOSYN-PWY Relationships: is a type of trypanothione metabolic process [GO:0046206]; is a type of glutathione derivative biosynthetic process [GO:1901687] Also known as: trypanothione anabolism, trypanothione biosynthesis, trypanothione formation, trypanothione synthesis